{
  "gene_symbol": "ARL6IP4",
  "gene": "UniProtKB:Q66PJ3",
  "term_id": "UNKNOWN:0001",
  "gene_name": "ADP-ribosylation factor-like protein 6-interacting protein 4",
  "term_label": "Unknown molecular function"
}